{
  "gene": "UniProtKB:Q7Z6J8",
  "gene_name": "E3 ubiquitin-protein ligase E3D",
  "term_label": "cyclin binding",
  "gene_symbol": "UBE3D",
  "term_id": "GO:0030332"
}